{
  "gene_symbol": "NPIPB12",
  "gene_name": "Nuclear pore complex-interacting protein family member B12",
  "gene": "UniProtKB:F8W0I5",
  "term_id": "UNKNOWN:0001",
  "term_label": "Unknown molecular function"
}